{
  "gene_name": "Cardiotrophin-like cytokine factor 1",
  "gene_symbol": "CLCF1",
  "term_id": "GO:0097058",
  "gene": "UniProtKB:Q9UBD9",
  "term_label": "CRLF-CLCF1 complex"
}